{
  "term_label": "heterotrimeric G-protein complex",
  "gene_name": "Guanine nucleotide-binding protein G(I)_G(S)_G(T) subunit beta-1",
  "term_id": "GO:0005834",
  "gene": "UniProtKB:P62873",
  "gene_symbol": "GNB1"
}